{
  "term_id": "GO:0052689",
  "gene_symbol": "ABHD5",
  "gene_name": "1-acylglycerol-3-phosphate O-acyltransferase ABHD5",
  "gene": "UniProtKB:Q8WTS1",
  "term_label": "carboxylic ester hydrolase activity"
}